single-stranded DNA exodeoxyribonuclease activity [GO:0008297] (molecular function) Sources: GOC:mah Also known as: single-stranded DNA specific exodeoxyribonuclease activity, ssDNA-specific exodeoxyribonuclease activity Relationships: is a type of DNA exonuclease activity, producing 5'-phosphomonoesters [GO:0016895] Subtypes: GO:0008310, single-stranded DNA 5'-3' DNA exonuclease activity [GO:0045145] Definition: Catalysis of the sequential cleavage of mononucleotides from a free 5' or 3' terminus of a single-stranded DNA molecule.